{
  "term_id": "GO:0034394",
  "gene_symbol": "GGA2",
  "gene_name": "ADP-ribosylation factor-binding protein GGA2",
  "term_label": "protein localization to cell surface",
  "gene": "UniProtKB:Q9UJY4"
}